{
  "term_id": "GO:0098632",
  "term_label": "cell-cell adhesion mediator activity",
  "gene_name": "Junctional adhesion molecule C",
  "gene_symbol": "JAM3",
  "gene": "UniProtKB:Q9BX67"
}